{
  "term_id": "GO:0005634",
  "gene": "UniProtKB:A7XYQ1",
  "gene_symbol": "SOBP",
  "gene_name": "Sine oculis-binding protein homolog",
  "term_label": "nucleus"
}